positive regulation of ubiquitin protein ligase activity [GO:1904668] (biological process) Definition: Any process that activates or increases the frequency, rate or extent of ubiquitin protein ligase activity. References: PMID:10921876, PMID:26216882 Sources: GOC:TermGenie, GOC:dph, GOC:vw, GO_REF:0000059 Also known as: positive regulation of protein ubiquitination activity, up regulation of protein ubiquitination activity, up regulation of ubiquitin ligase activity, up regulation of ubiquitin protein ligase activity, up-regulation of protein ubiquitination activity, up-regulation of ubiquitin ligase activity, up-regulation of ubiquitin protein ligase activity, upregulation of protein ubiquitination activity, upregulation of ubiquitin ligase activity, upregulation of ubiquitin protein ligase activity, activation of APC-Cdc20 complex activity, activation of APC-fizzy related complex activity, activation of anaphase-promoting complex activity, activation of protein ubiquitination activity, activation of ubiquitin ligase activity, activation of ubiquitin protein ligase activity, positive regulation of APC-fizzy related complex activity, up regulation of APC-fizzy related complex activity, up-regulation of APC-fizzy related complex activity, upregulation of APC-fizzy related complex activity, activation of E3, positive regulation of E3, positive regulation of ubiquitin ligase activity, up regulation of E3, up-regulation of E3, upregulation of E3 Relationships: is a type of positive regulation of ubiquitin-protein transferase activity [GO:0051443]; is a type of regulation of ubiquitin protein ligase activity [GO:1904666]; positively regulates ubiquitin protein ligase activity [GO:0061630]